{
  "gene_name": "Cytochrome P450 3A5",
  "gene": "UniProtKB:P20815",
  "term_label": "testosterone 6-beta-hydroxylase activity",
  "gene_symbol": "CYP3A5",
  "term_id": "GO:0050649"
}